Wnt receptor activity [GO:0042813] (molecular function) Sources: GOC:go_curators Also known as: Wnt-activated receptor activity, frizzled receptor activity, frizzled-2 receptor activity Definition: Combining with a Wnt protein and transmitting the signal across the plasma membrane to initiate a change in cell activity. Relationships: is a type of transmembrane signaling receptor activity [GO:0004888]; is part of Wnt signaling pathway [GO:0016055]; has part Wnt-protein binding [GO:0017147]